phytochelatin 2 import into vacuole [GO:0036246] (biological process) Relationships: is a type of oligopeptide transmembrane transport [GO:0035672]; is a type of phytochelatin import into vacuole [GO:0071995] Also known as: PC2 import into vacuole Definition: The directed movement of phytochelatin 2 (PC2) into the vacuole. Phytochelatin 2 is a glutathione-related peptide composed of (gamma-Glu-Cys)n-Gly where n=2, and where the Glu and Cys residues are linked through a gamma-carboxylamide bond. References: PMID:19001374 Sources: GOC:al